{
  "gene": "UniProtKB:O14526",
  "gene_name": "F-BAR domain only protein 1",
  "term_label": "cytoplasm",
  "gene_symbol": "FCHO1",
  "term_id": "GO:0005737"
}